{
  "gene": "UniProtKB:Q9Y223",
  "term_label": "N-acylmannosamine kinase activity",
  "term_id": "GO:0009384",
  "gene_name": "Bifunctional UDP-N-acetylglucosamine 2-epimerase_N-acetylmannosamine kinase",
  "gene_symbol": "GNE"
}